{
  "term_label": "immune receptor activity",
  "gene_symbol": "KIR2DL5B",
  "gene_name": "Killer cell immunoglobulin-like receptor 2DL5B",
  "term_id": "GO:0140375",
  "gene": "UniProtKB:Q8NHK3"
}